cell envelope Sec protein transport complex [GO:0031522] (cellular component) Definition: A transmembrane protein complex involved in the translocation of proteins across the cytoplasmic membrane. In Gram-negative bacteria, Sec-translocated proteins are subsequently secreted via the type II, IV, or V secretion systems. Sec complex components include SecA, D, E, F, G, Y and YajC. References: PMID:15223057 Sources: GOC:mtg_sensu Also known as: Sec complex, Sec secretion complex, Sec translocation complex, plasma membrane Sec complex Note: Note that this term represents the protein complex involved in transport of proteins across the cytoplasmic membrane. For proteins involved in bacterial type II secretion across the outer membrane, consider annotating to 'type II protein secretion complex ; GO:0015628'. For proteins involved in Sec-complex dependent translocation into the eukaryotic endoplasmic reticulum, consider annotating to 'endoplasmic reticulum Sec complex ; GO:0031205'. Relationships: is a type of intracellular protein-containing complex [GO:0140535]